{
  "term_id": "GO:0033280",
  "gene_symbol": "CYP27B1",
  "term_label": "response to vitamin D",
  "gene_name": "25-hydroxyvitamin D-1 alpha hydroxylase, mitochondrial",
  "gene": "UniProtKB:O15528"
}